photoreceptor cell fate specification [GO:0043704] (BP) Sources: GOC:mtg_sensu Definition: The process in which a cell becomes capable of differentiating autonomously into a photoreceptor cell in an environment that is neutral with respect to the developmental pathway. Upon specification, the cell fate can be reversed. Relationships: is a type of neuron fate specification [GO:0048665]; is part of photoreceptor cell fate commitment [GO:0046552] Subtypes: retinal cone cell fate specification [GO:0042672], R8 cell fate specification [GO:0045464]